{
  "gene_name": "Adherens junction-associated protein 1",
  "gene_symbol": "AJAP1",
  "gene": "UniProtKB:Q9UKB5",
  "term_id": "GO:0009898",
  "term_label": "cytoplasmic side of plasma membrane"
}